{
  "gene": "UniProtKB:Q15431",
  "gene_symbol": "SYCP1",
  "term_id": "GO:0051878",
  "gene_name": "Synaptonemal complex protein 1",
  "term_label": "lateral element assembly"
}